granzyme A production [GO:0035746] (biological process) Definition: The appearance of granzyme A due to biosynthesis or secretion following a cellular stimulus, resulting in an increase in its intracellular or extracellular levels. Note: Note that this term is in the subset of terms that should not be used for direct gene product annotation. Instead, select one of the 'regulation' children terms. Sources: GOC:BHF Regulation: regulated by regulation of granzyme A production [GO:2000511]; negatively regulated by negative regulation of granzyme A production [GO:2000512]; positively regulated by positive regulation of granzyme A production [GO:2000513] Relationships: is_a production of molecular mediator of immune response [GO:0002440]